indole-3-pyruvate monooxygenase activity [GO:0103075] (molecular function) Relationships: is a type of oxidoreductase activity, acting on paired donors, with incorporation or reduction of molecular oxygen, NAD(P)H as one donor, and incorporation of one atom of oxygen [GO:0016709] Sources: EC:1.14.13.168, GOC:pz Definition: Catalysis of the reaction: 3-(indol-3-yl)pyruvate + NADPH + O2 + H+ = indole-3-acetate + carbon dioxide + NADP + H2O.